{
  "gene_name": "Baculoviral IAP repeat-containing protein 5",
  "gene": "UniProtKB:O15392",
  "gene_symbol": "BIRC5",
  "term_id": "GO:0051233",
  "term_label": "spindle midzone"
}